{
  "gene_symbol": "LGALS9C",
  "gene": "UniProtKB:Q6DKI2",
  "term_id": "GO:0030246",
  "gene_name": "Galectin-9C",
  "term_label": "carbohydrate binding"
}